{
  "term_label": "immune response",
  "term_id": "GO:0006955",
  "gene_name": "Immunoglobulin kappa variable 1D-33",
  "gene": "UniProtKB:P01593",
  "gene_symbol": "IGKV1D-33"
}